{
  "gene": "UniProtKB:A0ZSE6",
  "gene_symbol": "TMEM30CP",
  "term_label": "Unknown molecular function",
  "term_id": "UNKNOWN:0001",
  "gene_name": "Cell cycle control protein 50C"
}